{
  "gene_symbol": "DNAJB2",
  "gene": "UniProtKB:P25686",
  "term_label": "ATPase activator activity",
  "gene_name": "DnaJ homolog subfamily B member 2",
  "term_id": "GO:0001671"
}